{
  "gene": "UniProtKB:P59533",
  "term_id": "GO:0001580",
  "gene_symbol": "TAS2R38",
  "gene_name": "Taste receptor type 2 member 38",
  "term_label": "detection of chemical stimulus involved in sensory perception of bitter taste"
}